{
  "gene_symbol": "CCL26",
  "term_id": "GO:0008009",
  "gene": "UniProtKB:Q9Y258",
  "gene_name": "C-C motif chemokine 26",
  "term_label": "chemokine activity"
}